{
  "gene_symbol": "BHLHA15",
  "gene_name": "Class A basic helix-loop-helix protein 15",
  "term_id": "GO:0061564",
  "gene": "UniProtKB:Q7RTS1",
  "term_label": "axon development"
}